{
  "gene_symbol": "MYH2",
  "gene_name": "Myosin-2",
  "gene": "UniProtKB:Q9UKX2",
  "term_label": "myosin filament",
  "term_id": "GO:0032982"
}